{
  "gene_symbol": "PLG",
  "term_label": "extracellular space",
  "gene_name": "Plasminogen",
  "gene": "UniProtKB:P00747",
  "term_id": "GO:0005615"
}